{
  "gene": "UniProtKB:Q13591",
  "gene_name": "Semaphorin-5A",
  "term_id": "GO:0007411",
  "gene_symbol": "SEMA5A",
  "term_label": "axon guidance"
}